{
  "gene": "UniProtKB:P24278",
  "term_label": "nucleoplasm",
  "gene_symbol": "ZBTB25",
  "gene_name": "Zinc finger and BTB domain-containing protein 25",
  "term_id": "GO:0005654"
}